{
  "term_id": "GO:0005200",
  "gene": "UniProtKB:Q9BQE3",
  "gene_symbol": "TUBA1C",
  "gene_name": "Tubulin alpha-1C chain",
  "term_label": "structural constituent of cytoskeleton"
}